{
  "gene_name": "Potassium voltage-gated channel subfamily KQT member 4",
  "term_id": "GO:0005249",
  "gene": "UniProtKB:P56696",
  "gene_symbol": "KCNQ4",
  "term_label": "voltage-gated potassium channel activity"
}